{
  "gene_symbol": "CCDC180",
  "term_id": "UNKNOWN:0001",
  "term_label": "Unknown molecular function",
  "gene_name": "Coiled-coil domain-containing protein 180",
  "gene": "UniProtKB:Q9P1Z9"
}